{
  "gene_symbol": "ALG5",
  "gene": "UniProtKB:Q9Y673",
  "gene_name": "Dolichyl-phosphate beta-glucosyltransferase",
  "term_id": "GO:0004581",
  "term_label": "dolichyl-phosphate beta-glucosyltransferase activity"
}